negative regulation of T cell activation [GO:0050868] (biological process) Also known as: down regulation of T cell activation, down-regulation of T cell activation, downregulation of T cell activation, negative regulation of T lymphocyte activation, negative regulation of T-cell activation, negative regulation of T-lymphocyte activation, inhibition of T cell activation Relationships: is a type of regulation of T cell activation [GO:0050863]; is a type of GO:0051250; is a type of GO:1903038; negatively regulates GO:0042110 Sources: GOC:ai Subtypes: negative regulation of T cell proliferation [GO:0042130], negative regulation of T cell differentiation [GO:0045581], negative regulation of alpha-beta T cell activation [GO:0046636], negative regulation of gamma-delta T cell activation [GO:0046644], negative regulation of establishment of T cell polarity [GO:1903904], negative regulation of T cell activation via T cell receptor contact with antigen bound to MHC molecule on antigen presenting cell [GO:2001189] Definition: Any process that stops, prevents, or reduces the frequency, rate or extent of T cell activation.